activated CD4-positive, alpha-beta T cell apoptotic process [GO:1905398] (biological process) Definition: Any apoptotic process in an activated CD4-positive, alpha-beta T cell. References: PMID:24187568 Sources: GOC:TermGenie, GO_REF:0000085 Also known as: activated CD4-positive, alpha-beta T lymphocyte apoptotic process, activated CD4-positive, alpha-beta T-cell apoptotic process, activated CD4-positive, alpha-beta T-lymphocyte apoptotic process, activated CD4-positive, alpha-beta T cell apoptosis, activated CD4-positive, alpha-beta T lymphocyte apoptosis, activated CD4-positive, alpha-beta T-cell apoptosis, activated CD4-positive, alpha-beta T-lymphocyte apoptosis Relationships: is a type of T cell apoptotic process [GO:0070231] Regulation: RO_0002211 by regulation of activated CD4-positive, alpha-beta T cell apoptotic process [GO:1905399]; negatively regulated by negative regulation of activated CD4-positive, alpha-beta T cell apoptotic process [GO:1905400]; RO_0002213 by GO:1905401